{
  "term_id": "UNKNOWN:0003",
  "gene_name": "T cell receptor alpha variable 26-1",
  "term_label": "Unknown cellular component",
  "gene": "UniProtKB:A0A087WT03",
  "gene_symbol": "TRAV26-1"
}